2-methyl-6-phytyl-1,4-benzoquinone methyltransferase activity [GO:0051741] (molecular function) Definition: Catalysis of the reaction: 2-methyl-6-phytyl-1,4-benzoquinone + S-adenosyl-methionine = 2,3-dimethyl-6-phytyl-1,4-benzoquinone + S-adenosyl-homocysteine. Relationships: is a type of S-adenosylmethionine-dependent methyltransferase activity [GO:0008757] Also known as: MPBQ methyltransferase activity Sources: MetaCyc:RXN-2542